meristem development [GO:0048507] (biological process) Sources: GOC:jid Regulation: regulated by regulation of meristem development [GO:0048509] Definition: The process whose specific outcome is the progression of the meristem over time, from its formation to the mature structure. Relationships: is_a tissue development [GO:0009888] Subtypes: GO:0048508, plantlet formation on parent plant [GO:0048624], shoot apical meristem development [GO:1902182]